cytokine-mediated signaling pathway [GO:0019221] (biological process) Subtypes: tumor necrosis factor-mediated signaling pathway [GO:0033209], leptin-mediated signaling pathway [GO:0033210], adiponectin-activated signaling pathway [GO:0033211], interleukin-18-mediated signaling pathway [GO:0035655], GO:0035691, interleukin-12-mediated signaling pathway [GO:0035722], interleukin-15-mediated signaling pathway [GO:0035723], interleukin-4-mediated signaling pathway [GO:0035771], interleukin-13-mediated signaling pathway [GO:0035772], interleukin-5-mediated signaling pathway [GO:0038043], GO:0038109, interleukin-2-mediated signaling pathway [GO:0038110], interleukin-7-mediated signaling pathway [GO:0038111], interleukin-8-mediated signaling pathway [GO:0038112], interleukin-9-mediated signaling pathway [GO:0038113], interleukin-21-mediated signaling pathway [GO:0038114], macrophage colony-stimulating factor signaling pathway [GO:0038145], interleukin-11-mediated signaling pathway [GO:0038154], GO:0038155, interleukin-3-mediated signaling pathway [GO:0038156], granulocyte-macrophage colony-stimulating factor signaling pathway [GO:0038157], granulocyte colony-stimulating factor signaling pathway [GO:0038158], prolactin signaling pathway [GO:0038161], erythropoietin-mediated signaling pathway [GO:0038162], GO:0038165, interleukin-33-mediated signaling pathway [GO:0038172], interleukin-17A-mediated signaling pathway [GO:0038173], interleukin-34-mediated signaling pathway [GO:0061514], chemokine-mediated signaling pathway [GO:0070098], interleukin-6-mediated signaling pathway [GO:0070102], GO:0070106, ciliary neurotrophic factor-mediated signaling pathway [GO:0070120], interleukin-1-mediated signaling pathway [GO:0070498], interleukin-35-mediated signaling pathway [GO:0070757], interleukin-32-mediated signaling pathway [GO:0097399], interleukin-17-mediated signaling pathway [GO:0097400], interleukin-10-mediated signaling pathway [GO:0140105], GO:0140854, interleukin-22-mediated signaling pathway [GO:0140865], interleukin-20-mediated signaling pathway [GO:0140866], GO:0140888 Definition: The series of molecular signals initiated by the binding of a cytokine to a receptor on the surface of a cell, and ending with the regulation of a downstream cellular process, e.g. transcription. Also known as: cytokine and chemokine mediated signaling pathway, cytokine mediated signalling pathway Regulation: regulated by regulation of cytokine-mediated signaling pathway [GO:0001959]; negatively regulated by negative regulation of cytokine-mediated signaling pathway [GO:0001960]; positively regulated by GO:0001961 References: PMID:19295629 Sources: GOC:mah, GOC:signaling Relationships: is a type of cell surface receptor signaling pathway [GO:0007166]; is part of GO:0071345